{
  "gene_name": "Tyrosine-protein phosphatase non-receptor type 5",
  "gene_symbol": "PTPN5",
  "term_label": "signal transduction",
  "gene": "UniProtKB:P54829",
  "term_id": "GO:0007165"
}